{
  "gene_symbol": "TP73",
  "term_label": "promoter-specific chromatin binding",
  "term_id": "GO:1990841",
  "gene_name": "Tumor protein p73",
  "gene": "UniProtKB:O15350"
}